{
  "term_id": "GO:0005829",
  "gene": "UniProtKB:P00568",
  "gene_symbol": "AK1",
  "gene_name": "Adenylate kinase isoenzyme 1",
  "term_label": "cytosol"
}